vascular endothelial cell response to laminar fluid shear stress [GO:0097700] (biological process) Definition: Any response to laminar fluid shear stress in a vascular endothelial cell. Relationships: is a type of cellular response to laminar fluid shear stress [GO:0071499]; is a type of vascular endothelial cell response to fluid shear stress [GO:0097699] References: PMID:21768538 Sources: GOC:BHF, GOC:BHF_miRNA, GOC:bc Also known as: blood vessel endothelial cell response to laminar fluid shear stress